superoxide-generating NADPH oxidase activity [GO:0106292] (molecular function) Definition: Catalysis of the reaction: NADPH + 2 O2 = H+ + NADP+ + 2 superoxide. Sources: RHEA:63180 Relationships: is a type of superoxide-generating NAD(P)H oxidase activity [GO:0016175] Regulation: positively regulated by superoxide-generating NADPH oxidase activator activity [GO:0016176]